{
  "term_label": "cell differentiation",
  "gene_symbol": "ETV3L",
  "term_id": "GO:0030154",
  "gene": "UniProtKB:Q6ZN32",
  "gene_name": "ETS translocation variant 3-like protein"
}